{
  "term_id": "UNKNOWN:0003",
  "gene": "UniProtKB:A0A1B0GV96",
  "gene_symbol": "CHD9NB",
  "term_label": "Unknown cellular component",
  "gene_name": "CHD9 neighbor protein"
}